{
  "term_id": "GO:0038023",
  "gene_symbol": "LINGO3",
  "gene": "UniProtKB:P0C6S8",
  "term_label": "signaling receptor activity",
  "gene_name": "Leucine-rich repeat and immunoglobulin-like domain-containing nogo receptor-interacting protein 3"
}